pullulanase activity [GO:0051060] (molecular function) Definition: Catalysis of the hydrolysis of (1,6)-alpha-D-glucosidic linkages in pullulan (a linear polymer of alpha-(1,6)-linked maltotriose units) and in amylopectin and glycogen, and the a- and b-limit dextrins of amylopectin and glycogen. Relationships: is a type of hydrolase activity, hydrolyzing O-glycosyl compounds [GO:0004553] Sources: EC:3.2.1.41 Also known as: debranching enzyme activity, alpha-dextrin endo-1,6-alpha-glucosidase activity, amylopectin 6-glucanohydrolase activity, pullulan 6-glucanohydrolase activity, R-enzyme, bacterial debranching enzyme, limit dextrinase, pullulan alpha-1,6-glucanohydrolase activity